{
  "gene_name": "Barrier-to-autointegration factor-like protein",
  "term_label": "DNA binding",
  "term_id": "GO:0003677",
  "gene": "UniProtKB:Q9H503",
  "gene_symbol": "BANF2"
}